{
  "gene": "UniProtKB:Q6ZSI9",
  "term_label": "calcium-dependent cysteine-type endopeptidase activity",
  "term_id": "GO:0004198",
  "gene_symbol": "CAPN12",
  "gene_name": "Calpain-12"
}